epinephrine biosynthetic process [GO:0042418] (biological process) Definition: The chemical reactions and pathways resulting in the formation of epinephrine, a hormone produced by the medulla of the adrenal glands that increases heart activity, improves the power and prolongs the action of muscles, and increases the rate and depth of breathing. It is synthesized by the methylation of norepinephrine. Sources: GOC:jl, ISBN:0192801023, ISBN:0198506732 Relationships: is a type of epinephrine metabolic process [GO:0042414]; is a type of GO:0042423 Also known as: adrenaline biosynthesis, adrenaline biosynthetic process, epinephrine anabolism, epinephrine biosynthesis, epinephrine formation, epinephrine synthesis